{
  "term_id": "GO:0005739",
  "term_label": "mitochondrion",
  "gene_symbol": "ANTKMT",
  "gene": "UniProtKB:Q9BQD7",
  "gene_name": "Adenine nucleotide translocase lysine N-methyltransferase"
}